positive regulation of viral DNA genome packaging via site-specific sequence recognition [GO:1905138] (biological process) Also known as: up regulation of viral DNA genome packaging via site-specific sequence recognition, up-regulation of viral DNA genome packaging via site-specific sequence recognition, upregulation of viral DNA genome packaging via site-specific sequence recognition, activation of viral DNA genome packaging via site-specific sequence recognition Definition: Any process that activates or increases the frequency, rate or extent of viral DNA genome packaging via site-specific sequence recognition. Relationships: is a type of positive regulation of viral life cycle [GO:1903902]; is a type of regulation of viral DNA genome packaging via site-specific sequence recognition [GO:1905137]; positively regulates viral DNA genome packaging via site-specific sequence recognition [GO:0098035] References: PMID:24711378 Sources: GOC:TermGenie, GO_REF:0000058